{
  "term_id": "GO:0032801",
  "gene_symbol": "MVB12A",
  "gene_name": "Multivesicular body subunit 12A",
  "term_label": "receptor catabolic process",
  "gene": "UniProtKB:Q96EY5"
}